{
  "gene_symbol": "ZNF580",
  "gene": "UniProtKB:Q9UK33",
  "term_label": "DNA-binding transcription activator activity, RNA polymerase II-specific",
  "term_id": "GO:0001228",
  "gene_name": "Zinc finger protein 580"
}